{
  "term_id": "GO:0005886",
  "gene_symbol": "CASK",
  "gene_name": "Peripheral plasma membrane protein CASK",
  "gene": "UniProtKB:O14936",
  "term_label": "plasma membrane"
}